butyrate catabolic process [GO:0046359] (biological process) Definition: The chemical reactions and pathways resulting in the breakdown of butyrate, the anion of butyric acid. Sources: ISBN:0198506732 Also known as: butanoic acid breakdown, butanoic acid catabolic process, butanoic acid catabolism, butanoic acid degradation, butyrate breakdown, butyrate catabolism, butyrate degradation Relationships: is a type of GO:0019605; is a type of short-chain fatty acid catabolic process [GO:0019626]